{
  "gene_name": "Small integral membrane protein 18",
  "term_id": "UNKNOWN:0003",
  "term_label": "Unknown cellular component",
  "gene": "UniProtKB:P0DKX4",
  "gene_symbol": "SMIM18"
}